{
  "gene_symbol": "ATP9A",
  "gene_name": "Probable phospholipid-transporting ATPase IIA",
  "term_id": "GO:0005802",
  "term_label": "trans-Golgi network",
  "gene": "UniProtKB:O75110"
}